{
  "gene": "UniProtKB:Q86Z02",
  "term_id": "GO:0004713",
  "gene_name": "Homeodomain-interacting protein kinase 1",
  "term_label": "protein tyrosine kinase activity",
  "gene_symbol": "HIPK1"
}